{
  "gene_symbol": "CUL4B",
  "gene": "UniProtKB:Q13620",
  "term_id": "GO:0043161",
  "term_label": "proteasome-mediated ubiquitin-dependent protein catabolic process",
  "gene_name": "Cullin-4B"
}